{
  "gene_symbol": "GOPC",
  "term_id": "GO:0030140",
  "gene": "UniProtKB:Q9HD26",
  "term_label": "trans-Golgi network transport vesicle",
  "gene_name": "Golgi-associated PDZ and coiled-coil motif-containing protein"
}